{
  "gene_symbol": "SLC16A1",
  "gene_name": "Monocarboxylate transporter 1",
  "gene": "UniProtKB:P53985",
  "term_label": "plasma membrane lactate transport",
  "term_id": "GO:0035879"
}